{
  "gene_symbol": "POLA2",
  "term_id": "GO:0006270",
  "term_label": "DNA replication initiation",
  "gene_name": "DNA polymerase alpha subunit B",
  "gene": "UniProtKB:Q14181"
}